regulation of anthocyanin biosynthetic process [GO:0031540] (biological process) Definition: Any process that modulates the frequency, rate or extent of the chemical reactions and pathways resulting in the formation of anthocyanins. Relationships: is a type of regulation of flavonoid biosynthetic process [GO:0009962]; is a type of regulation of anthocyanin metabolic process [GO:0031537]; regulates anthocyanin-containing compound biosynthetic process [GO:0009718] Sources: GOC:mah Subtypes: negative regulation of anthocyanin biosynthetic process [GO:0031541], GO:0031542 Also known as: regulation of anthocyanin anabolism, regulation of anthocyanin biosynthesis, regulation of anthocyanin formation, regulation of anthocyanin synthesis